{
  "gene_symbol": "FXR1",
  "term_label": "mRNA 3'-UTR binding",
  "gene_name": "RNA-binding protein FXR1",
  "gene": "UniProtKB:P51114",
  "term_id": "GO:0003730"
}